{
  "term_label": "Unknown biological process",
  "gene_symbol": "OR4K1",
  "gene": "UniProtKB:Q8NGD4",
  "term_id": "UNKNOWN:0002",
  "gene_name": "Olfactory receptor 4K1"
}